{
  "gene_symbol": "CPNE6",
  "term_id": "GO:0005886",
  "term_label": "plasma membrane",
  "gene_name": "Copine-6",
  "gene": "UniProtKB:O95741"
}